17-beta-hydroxysteroid dehydrogenase (NADP+) activity [GO:0072582] (molecular function) Subtypes: testosterone dehydrogenase (NADP+) activity [GO:0047045] Definition: Catalysis of the reaction: a 17-beta-hydroxysteroid + NADP+ = a 17-oxosteroid + NADPH + H+. References: PMID:17074428 Sources: GOC:kad Relationships: is a type of steroid dehydrogenase activity, acting on the CH-OH group of donors, NAD or NADP as acceptor [GO:0033764]